{
  "gene_name": "Succinyl-CoA:3-ketoacid coenzyme A transferase 1, mitochondrial",
  "gene": "UniProtKB:P55809",
  "term_id": "GO:1902224",
  "term_label": "ketone body metabolic process",
  "gene_symbol": "OXCT1"
}